canonical Wnt signaling pathway involved in positive regulation of apoptotic process [GO:0044337] (biological process) Also known as: canonical Wnt receptor signaling pathway involved in positive regulation of apoptotic process, canonical Wnt receptor signalling pathway involved in positive regulation of apoptosis, canonical Wnt-activated signaling pathway involved in positive regulation of apoptotic process, canonical Wnt receptor signaling pathway involved in positive regulation of apoptosis Sources: GOC:BHF, GOC:jl, GOC:mtg_apoptosis Definition: The series of molecular signals initiated by binding of a Wnt protein to a frizzled family receptor on the surface of the target cell, followed by propagation of the signal via beta-catenin, and ending with a change in transcription of target genes involved in the positive regulation of apoptotic process. Relationships: is a type of canonical Wnt signaling pathway [GO:0060070]; is part of positive regulation of apoptotic process [GO:0043065]